{
  "gene": "UniProtKB:O60673",
  "term_label": "DNA-directed DNA polymerase activity",
  "gene_symbol": "REV3L",
  "gene_name": "DNA polymerase zeta catalytic subunit",
  "term_id": "GO:0003887"
}